monomethylamine methyltransferase activity [GO:0043852] (molecular function) References: PMID:9195968 Relationships: is a type of methyltransferase activity [GO:0008168] Definition: Catalysis of the reaction: monomethylamine + a monomethylamine corrinoid protein = a methylated monomethylamine corrinoid protein + NH3. Note: This function is the first step in the pathway of methanogenesis from monomethylamine. Also known as: monomethylamine:corrinoid methyltransferase activity, MMAMT, MtmB